IRES-dependent translational initiation of linear mRNA [GO:0002192] (biological process) Relationships: is a type of cap-independent translational initiation of linear mRNA [GO:0110017]; has part IRES-mediated translation initiation factor activity [GO:0160297] Definition: The process where translation initiation recruits the 40S ribosomal subunits via an internal ribosome entry segment (IRES) before an AUG codon is encountered in an appropriate sequence context to initiate linear mRNA translation. References: PMID:17284590